glucose-1-phosphate thymidylyltransferase activity [GO:0008879] (molecular function) Definition: Catalysis of the reaction: alpha-D-glucose 1-phosphate + dTTP = diphosphate + dTDP-glucose. Sources: EC:2.7.7.24, RHEA:15225 Also known as: TDP-glucose pyrophosphorylase activity, dTDP-glucose diphosphorylase activity, dTDP-glucose pyrophosphorylase activity, dTDP-glucose synthase activity, dTTP:alpha-D-glucose-1-phosphate thymidylyltransferase activity, glucose 1-phosphate thymidylyltransferase activity, thymidine diphosphate glucose pyrophosphorylase activity, thymidine diphosphoglucose pyrophosphorylase activity Relationships: is a type of nucleotidyltransferase activity [GO:0016779]